{
  "term_id": "GO:0038023",
  "gene": "UniProtKB:Q6UXK5",
  "gene_name": "Leucine-rich repeat neuronal protein 1",
  "gene_symbol": "LRRN1",
  "term_label": "signaling receptor activity"
}